{
  "gene_name": "Putative uncharacterized protein LINC02908",
  "term_label": "Unknown biological process",
  "gene": "UniProtKB:Q6ZV77",
  "term_id": "UNKNOWN:0002",
  "gene_symbol": "LINC02908"
}